{
  "gene_symbol": "KLF1",
  "gene_name": "Krueppel-like factor 1",
  "term_label": "regulation of transcription by RNA polymerase II",
  "gene": "UniProtKB:Q13351",
  "term_id": "GO:0006357"
}